cyclohexylsulfamate metabolic process [GO:0018892] (biological process) Also known as: cyclohexylsulfamate metabolism, cyclohexylsulphamate metabolic process, cyclohexylsulphamate metabolism Definition: The chemical reactions and pathways involving cyclohexylsulfamate, also known as cyclamic acid. Sodium cyclohexylsulfamate (CHS-Na) was a widely used sweetening agent but was banned because of the suspicion of carcinogenicity and metabolic conversion to cyclohexylamine (CHA), a toxic substance. It is now used as a fungicide. Sources: UM-BBD_pathwayID:chs Relationships: is a type of sulfur compound metabolic process [GO:0006790]; is a type of xenobiotic metabolic process [GO:0006805]; is a type of oxoacid metabolic process [GO:0043436]